{
  "term_label": "positive regulation of canonical Wnt signaling pathway",
  "term_id": "GO:0090263",
  "gene_name": "Protein phosphatase 1B",
  "gene": "UniProtKB:O75688",
  "gene_symbol": "PPM1B"
}